{
  "gene_name": "NTPase KAP family P-loop domain-containing protein 1",
  "term_id": "UNKNOWN:0001",
  "gene": "UniProtKB:Q17RQ9",
  "term_label": "Unknown molecular function",
  "gene_symbol": "NKPD1"
}